prostaglandin F2-alpha receptor binding [GO:0031868] (molecular function) Also known as: prostanoid FP receptor binding, prostaglandin F2-alpha receptor ligand Definition: Binding to a prostaglandin F2-alpha receptor. Sources: GOC:mah, GOC:nln Relationships: is a type of prostanoid receptor binding [GO:0031862]